{
  "gene_symbol": "RPP38-DT",
  "term_id": "UNKNOWN:0001",
  "gene": "UniProtKB:Q8N326",
  "gene_name": "Putative uncharacterized protein RPP38-DT",
  "term_label": "Unknown molecular function"
}